{
  "gene_name": "Potassium channel subfamily K member 10",
  "term_label": "potassium ion leak channel activity",
  "gene": "UniProtKB:P57789",
  "gene_symbol": "KCNK10",
  "term_id": "GO:0022841"
}